{
  "gene": "UniProtKB:Q9BYV1",
  "gene_symbol": "AGXT2",
  "gene_name": "Alanine--glyoxylate aminotransferase 2, mitochondrial",
  "term_label": "mitochondrion",
  "term_id": "GO:0005739"
}